regulation of spindle elongation [GO:0032887] (biological process) Definition: Any process that modulates the frequency, rate or extent of the cell cycle process in which the distance is lengthened between poles of the spindle. Subtypes: regulation of mitotic spindle elongation [GO:0032888], regulation of meiotic spindle elongation [GO:1902119] Relationships: is_a regulation of cell cycle process [GO:0010564]; is a type of regulation of microtubule-based process [GO:0032886]; regulates GO:0051231 Sources: GOC:mah